anaerobic L-phenylalanine oxidation [GO:0019561] (biological process) Sources: GOC:mah, MetaCyc:ANAPHENOXI-PWY Definition: The chemical reactions and pathways resulting in the breakdown of L-phenylalanine under anaerobic conditions; occurs via the intermediates phenylpyruvate and phenylacetaldehyde. Relationships: is a type of L-phenylalanine catabolic process [GO:0006559]